{
  "gene_name": "Protein FAM241B",
  "gene_symbol": "FAM241B",
  "term_label": "Unknown biological process",
  "term_id": "UNKNOWN:0002",
  "gene": "UniProtKB:Q96D05"
}